{
  "gene_name": "Transmembrane protein 265",
  "term_label": "Unknown cellular component",
  "gene": "UniProtKB:A0A087WTH1",
  "term_id": "UNKNOWN:0003",
  "gene_symbol": "TMEM265"
}